{
  "gene_name": "P antigen family member 4",
  "term_id": "UNKNOWN:0003",
  "gene_symbol": "PAGE4",
  "gene": "UniProtKB:O60829",
  "term_label": "Unknown cellular component"
}